{
  "gene": "UniProtKB:Q9NVE7",
  "term_id": "GO:0016791",
  "gene_symbol": "PANK4",
  "gene_name": "4'-phosphopantetheine phosphatase",
  "term_label": "phosphatase activity"
}